{
  "gene_name": "Methyl-CpG-binding domain protein 3-like 2",
  "term_label": "nucleus",
  "term_id": "GO:0005634",
  "gene": "UniProtKB:Q8NHZ7",
  "gene_symbol": "MBD3L2"
}